{
  "term_id": "GO:0005615",
  "gene_name": "Kallikrein-2",
  "gene_symbol": "KLK2",
  "term_label": "extracellular space",
  "gene": "UniProtKB:P20151"
}